{
  "gene": "UniProtKB:O60333",
  "term_id": "GO:0008017",
  "gene_name": "Kinesin-like protein KIF1B",
  "gene_symbol": "KIF1B",
  "term_label": "microtubule binding"
}